{
  "term_label": "mRNA 3'-end processing",
  "gene": "UniProtKB:Q5VT52",
  "term_id": "GO:0031124",
  "gene_symbol": "RPRD2",
  "gene_name": "Regulation of nuclear pre-mRNA domain-containing protein 2"
}